{
  "term_label": "Unknown biological process",
  "term_id": "UNKNOWN:0002",
  "gene_name": "Centromere protein V-like protein 2",
  "gene": "UniProtKB:P0DPI3",
  "gene_symbol": "CENPVL2"
}